ribokinase activity [GO:0004747] (molecular function) Also known as: ATP:D-ribose 5-phosphotransferase activity, D-ribokinase activity, deoxyribokinase activity, ribokinase (phosphorylating) Definition: Catalysis of the reaction: ATP + D-ribose = ADP + D-ribose 5-phosphate. Relationships: is a type of phosphotransferase activity, alcohol group as acceptor [GO:0016773]; is a type of carbohydrate kinase activity [GO:0019200] Sources: EC:2.7.1.15